malolactic fermentation [GO:0043464] (biological process) References: PMID:10427020, PMID:8808948 Definition: The anaerobic enzymatic conversion of L-malate to L-lactate and carbon dioxide, yielding energy in the form of ATP. Relationships: is a type of GO:0006113 Also known as: L-malate fermentation, malate fermentation, malo-lactate fermentation, malolactate fermentation